iron ion binding [GO:0005506] (molecular function) Sources: GOC:ai Relationships: is a type of transition metal ion binding [GO:0046914] Also known as: iron binding Subtypes: GO:0008198, ferric iron binding [GO:0008199] Definition: Binding to an iron (Fe) ion.